{
  "gene_symbol": "GOLGA7B",
  "term_label": "protein targeting to membrane",
  "gene": "UniProtKB:Q2TAP0",
  "term_id": "GO:0006612",
  "gene_name": "Golgin subfamily A member 7B"
}